{
  "gene_name": "Peptidyl-prolyl cis-trans isomerase A-like 4F",
  "gene": "UniProtKB:P0DN26",
  "gene_symbol": "PPIAL4F",
  "term_label": "protein folding",
  "term_id": "GO:0006457"
}